negative regulation of skeletal muscle tissue growth [GO:0048632] (biological process) Definition: Any process that stops, prevents, or reduces the frequency, rate or extent of skeletal muscle growth. Also known as: down regulation of skeletal muscle growth, down-regulation of skeletal muscle growth, downregulation of skeletal muscle growth, inhibition of skeletal muscle growth References: PMID:15726494, PMID:15907921 Sources: GOC:lm Relationships: is a type of regulation of skeletal muscle tissue growth [GO:0048631]; is a type of negative regulation of developmental growth [GO:0048640]; negatively regulates skeletal muscle tissue growth [GO:0048630]